{
  "term_label": "cell surface receptor protein serine/threonine kinase signaling pathway",
  "gene_name": "Inhibin beta E chain",
  "gene_symbol": "INHBE",
  "term_id": "GO:0007178",
  "gene": "UniProtKB:P58166"
}